{
  "term_id": "UNKNOWN:0001",
  "gene_name": "Type 2 DNA topoisomerase 6 subunit B-like",
  "gene_symbol": "TOP6BL",
  "gene": "UniProtKB:Q8N6T0",
  "term_label": "Unknown molecular function"
}